{
  "gene_symbol": "GNPDA2",
  "gene": "UniProtKB:Q8TDQ7",
  "term_id": "GO:0004342",
  "term_label": "glucosamine-6-phosphate deaminase activity",
  "gene_name": "Glucosamine-6-phosphate isomerase 2"
}